{
  "gene_symbol": "CEL",
  "term_label": "pancreatic juice secretion",
  "term_id": "GO:0030157",
  "gene": "UniProtKB:P19835",
  "gene_name": "Bile salt-activated lipase"
}